{
  "term_label": "IgG receptor activity",
  "gene": "UniProtKB:P12314",
  "term_id": "GO:0019770",
  "gene_symbol": "FCGR1A",
  "gene_name": "High affinity immunoglobulin gamma Fc receptor I"
}